cleavage apparatus septin structure [GO:0032161] (CC) Subtypes: cellular bud neck septin ring [GO:0000144], prospore septin ring [GO:0032169], GO:0032174, cellular bud neck split septin rings [GO:0032177], medial cortex septin ring [GO:0036391] Relationships: is a type of GO:0110165; is part of GO:0005938; is part of cell division site [GO:0032153]; is part of septin cytoskeleton [GO:0032156] Definition: Any of a series of structures composed of septins and septin-associated proteins localized to the cleavage plane which are involved in cytokinesis. References: PMID:12101122, PMID:15774761, PMID:16009555 Sources: GOC:krc